{
  "gene": "UniProtKB:Q96JE7",
  "term_id": "GO:0070973",
  "term_label": "protein localization to endoplasmic reticulum exit site",
  "gene_symbol": "SEC16B",
  "gene_name": "Protein transport protein Sec16B"
}